{
  "gene_name": "Protein FAM170B",
  "term_label": "Unknown molecular function",
  "gene": "UniProtKB:A6NMN3",
  "term_id": "UNKNOWN:0001",
  "gene_symbol": "FAM170B"
}